{
  "term_id": "UNKNOWN:0001",
  "gene": "UniProtKB:Q9H4E7",
  "gene_symbol": "DEF6",
  "term_label": "Unknown molecular function",
  "gene_name": "Differentially expressed in FDCP 6 homolog"
}